{
  "gene_symbol": "KLHDC7B",
  "term_label": "Unknown cellular component",
  "gene": "UniProtKB:Q96G42",
  "gene_name": "Kelch domain-containing protein 7B",
  "term_id": "UNKNOWN:0003"
}